{
  "gene": "UniProtKB:H3BQL2",
  "term_id": "GO:0032580",
  "gene_symbol": "GOLGA8T",
  "gene_name": "Golgin subfamily A member 8T",
  "term_label": "Golgi cisterna membrane"
}